{
  "gene_symbol": "COX20",
  "term_label": "Unknown molecular function",
  "term_id": "UNKNOWN:0001",
  "gene_name": "Cytochrome c oxidase assembly protein COX20, mitochondrial",
  "gene": "UniProtKB:Q5RI15"
}